{
  "gene": "UniProtKB:P10635",
  "gene_name": "Cytochrome P450 2D6",
  "term_id": "GO:0006805",
  "gene_symbol": "CYP2D6",
  "term_label": "xenobiotic metabolic process"
}